calcitonin gene-related peptide receptor activity [GO:0001635] (molecular function) References: PMID:12037140 Sources: GOC:mah Relationships: is a type of calcitonin family receptor activity [GO:0097642] Also known as: CGRP receptor, calcitonin gene-related polypeptide receptor activity Definition: Combining with a calcitonin gene-related polypeptide (CGRP) to initiate a change in cell activity.